{
  "gene": "UniProtKB:P36871",
  "term_id": "GO:0005975",
  "term_label": "carbohydrate metabolic process",
  "gene_name": "Phosphoglucomutase-1",
  "gene_symbol": "PGM1"
}